histone H3K4 deacetylase activity, NAD-dependent [GO:0141222] (molecular function) References: PMID:20299449, PMID:23771057 Relationships: is a type of histone deacetylase activity, NAD-dependent [GO:0017136]; is a type of GO:0141050 Definition: Catalysis of the reaction: histone H3 N6-acetyl-L-lysine (position 14) + NAD+ + H2O = histone H3 L-lysine (position 14) + 2''-O-acetyl-ADP-D-ribose + nicotinamide. This reaction transfers an acetyl group attached to a lysine residue in H3K4 to NAD, producing nicotinamide. Note: Comment: Note that the residue position corresponds to the canonical human H3 histone (UniProtKB:P84243); this residue is conserved across all eukaryotes. Residue 1 is the first residue following removal of the initiating Methionine (Met). Note that each histone is encoded by multiple genes, and sequences may vary across different genes within an organism.